{
  "gene_symbol": "MECOM",
  "term_id": "GO:0005634",
  "gene_name": "Histone-lysine N-methyltransferase MECOM",
  "gene": "UniProtKB:Q03112",
  "term_label": "nucleus"
}